{
  "gene_name": "Glutamate-rich protein 6",
  "term_label": "Unknown cellular component",
  "gene": "UniProtKB:Q7L0X2",
  "term_id": "UNKNOWN:0003",
  "gene_symbol": "ERICH6"
}